{
  "gene_symbol": "POU2F1",
  "gene_name": "POU domain, class 2, transcription factor 1",
  "term_label": "regulation of transcription by RNA polymerase II",
  "gene": "UniProtKB:P14859",
  "term_id": "GO:0006357"
}